{
  "term_id": "UNKNOWN:0001",
  "gene": "UniProtKB:Q3C1V1",
  "gene_symbol": "C11orf91",
  "gene_name": "Uncharacterized protein C11orf91",
  "term_label": "Unknown molecular function"
}